{
  "term_label": "extracellular space",
  "gene": "UniProtKB:P01286",
  "term_id": "GO:0005615",
  "gene_symbol": "GHRH",
  "gene_name": "Somatoliberin"
}